{
  "term_label": "visual perception",
  "gene_name": "Beta-crystallin A4",
  "gene_symbol": "CRYBA4",
  "term_id": "GO:0007601",
  "gene": "UniProtKB:P53673"
}